{
  "gene_symbol": "SEPTIN9",
  "term_id": "GO:0060090",
  "gene_name": "Septin-9",
  "term_label": "molecular adaptor activity",
  "gene": "UniProtKB:Q9UHD8"
}